hypoxanthine DNA N-glycosylase activity [GO:0097507] (MF) Also known as: hypoxanthine-DNA glycosylase activity Relationships: is a type of deaminated base DNA N-glycosylase activity [GO:0097506] Definition: DNA N-glycosylase activity acting on deaminated adenine (hypoxanthine). References: PMID:18789404 Sources: GOC:al